{
  "term_id": "GO:0048786",
  "gene": "UniProtKB:Q8ND30",
  "gene_name": "Liprin-beta-2",
  "gene_symbol": "PPFIBP2",
  "term_label": "presynaptic active zone"
}